RNA dihydrouridine synthase activity [GO:0106413] (molecular function) References: PMID:12581659, PMID:25073379 Definition: Catalysis of the reaction: RNA-uracil + NAD(P)+ = RNA-dihydrouridine + NAD(P)H + H+. Subtypes: tRNA dihydrouridine synthase activity [GO:0017150], mRNA dihydrouridine synthase activity [GO:0106414] Relationships: is a type of oxidoreductase activity, acting on the CH-CH group of donors, NAD or NADP as acceptor [GO:0016628]